{
  "term_id": "GO:0052651",
  "gene_name": "Protein ABHD16B",
  "term_label": "monoacylglycerol catabolic process",
  "gene": "UniProtKB:Q9H3Z7",
  "gene_symbol": "ABHD16B"
}